{
  "term_id": "UNKNOWN:0003",
  "gene_name": "Protein FAM209B",
  "gene": "UniProtKB:Q5JX69",
  "gene_symbol": "FAM209B",
  "term_label": "Unknown cellular component"
}